{
  "gene_name": "Zinc finger protein 695",
  "gene": "UniProtKB:Q8IW36",
  "term_label": "Unknown cellular component",
  "gene_symbol": "ZNF695",
  "term_id": "UNKNOWN:0003"
}